{
  "gene_symbol": "EDA2R",
  "gene_name": "Tumor necrosis factor receptor superfamily member 27",
  "term_id": "GO:0043123",
  "term_label": "positive regulation of canonical NF-kappaB signal transduction",
  "gene": "UniProtKB:Q9HAV5"
}